catecholamine secretion, neurotransmission [GO:0160043] (biological process) Definition: The regulated release of catecholamine by a cell in which the catecholamine acts as a neurotransmitter. References: PMID:10191060 Relationships: is a type of neurotransmitter secretion [GO:0007269]; is a type of catecholamine secretion [GO:0050432] Subtypes: dopamine secretion, neurotransmission [GO:0061527], epinephrine secretion, neurotransmission [GO:0061529], norepinephrine secretion, neurotransmission [GO:0061533]